{
  "term_id": "GO:0000062",
  "term_label": "fatty-acyl-CoA binding",
  "gene_name": "Acyl-CoA-binding domain-containing protein 5",
  "gene_symbol": "ACBD5",
  "gene": "UniProtKB:Q5T8D3"
}